{
  "gene": "UniProtKB:Q96PS6",
  "gene_symbol": "GAFA1",
  "term_id": "UNKNOWN:0002",
  "gene_name": "Putative uncharacterized protein GAFA-1",
  "term_label": "Unknown biological process"
}